{
  "gene": "UniProtKB:Q9NVR2",
  "term_label": "snRNA processing",
  "term_id": "GO:0016180",
  "gene_name": "Integrator complex subunit 10",
  "gene_symbol": "INTS10"
}